acute inflammatory response to antigenic stimulus [GO:0002438] (biological process) Sources: GOC:add, GO_REF:0000022, ISBN:0781735149 Subtypes: hypersensitivity [GO:0002524] Relationships: is a type of inflammatory response to antigenic stimulus [GO:0002437]; is a type of acute inflammatory response [GO:0002526] Definition: An acute inflammatory response to an antigenic stimulus. An acute inflammatory response occurs within a matter of minutes or hours, and either resolves within a few days or becomes a chronic inflammatory response. Regulation: RO_0002211 by regulation of acute inflammatory response to antigenic stimulus [GO:0002864]; negatively regulated by GO:0002865; positively regulated by GO:0002866